{
  "term_id": "GO:0060090",
  "gene_symbol": "APBB2",
  "gene": "UniProtKB:Q92870",
  "term_label": "molecular adaptor activity",
  "gene_name": "Amyloid beta precursor protein binding family B member 2"
}